{
  "term_label": "Unknown molecular function",
  "gene_name": "Putative serine_threonine-protein kinase SIK1B",
  "gene": "UniProtKB:A0A0B4J2F2",
  "term_id": "UNKNOWN:0001",
  "gene_symbol": "SIK1B"
}